{
  "gene_name": "Inosine triphosphate pyrophosphatase",
  "term_label": "cytoplasm",
  "term_id": "GO:0005737",
  "gene": "UniProtKB:Q9BY32",
  "gene_symbol": "ITPA"
}